{
  "gene_name": "Achaete-scute homolog 2",
  "term_label": "DNA-binding transcription factor activity, RNA polymerase II-specific",
  "gene": "UniProtKB:Q99929",
  "term_id": "GO:0000981",
  "gene_symbol": "ASCL2"
}